{
  "gene": "UniProtKB:Q712K3",
  "term_id": "GO:0006511",
  "term_label": "ubiquitin-dependent protein catabolic process",
  "gene_name": "Ubiquitin-conjugating enzyme E2 R2",
  "gene_symbol": "UBE2R2"
}